{
  "term_id": "UNKNOWN:0003",
  "gene_symbol": "A0A7I2V6D3",
  "gene": "UniProtKB:A0A7I2V6D3",
  "term_label": "Unknown cellular component",
  "gene_name": "Uncharacterized protein"
}